{
  "gene_name": "Leucine-rich repeat-containing protein 57",
  "term_label": "Unknown molecular function",
  "term_id": "UNKNOWN:0001",
  "gene_symbol": "LRRC57",
  "gene": "UniProtKB:Q8N9N7"
}